{
  "term_label": "Unknown molecular function",
  "gene_symbol": "UNQ9370_PRO34162",
  "term_id": "UNKNOWN:0001",
  "gene": "UniProtKB:Q6UXP9",
  "gene_name": "Putative uncharacterized protein UNQ9370_PRO34162"
}